{
  "gene_name": "E3 ubiquitin-protein ligase RNF4",
  "gene_symbol": "RNF4",
  "gene": "UniProtKB:P78317",
  "term_label": "PML body",
  "term_id": "GO:0016605"
}